{
  "gene_name": "Rhodopsin kinase GRK7",
  "gene_symbol": "GRK7",
  "gene": "UniProtKB:Q8WTQ7",
  "term_id": "GO:0050254",
  "term_label": "rhodopsin kinase activity"
}